{
  "term_label": "protein folding chaperone",
  "gene_name": "Heat shock-related 70 kDa protein 2",
  "gene": "UniProtKB:P54652",
  "gene_symbol": "HSPA2",
  "term_id": "GO:0044183"
}